negative stranded viral RNA transcription [GO:0039697] (biological process) Relationships: is a type of RNA-templated viral transcription [GO:0039696] Definition: A viral transcription process that uses negative stranded (-) single stranded (ss) RNA as a template. Sources: VZ:1096